{
  "term_id": "GO:1903830",
  "term_label": "magnesium ion transmembrane transport",
  "gene_symbol": "MAGT1",
  "gene_name": "Magnesium transporter protein 1",
  "gene": "UniProtKB:Q9H0U3"
}